response to anisomycin [GO:0072739] (biological process) Definition: Any process that results in a change in state or activity of a cell or an organism (in terms of movement, secretion, enzyme production, gene expression, etc.) as a result of an anisomycin stimulus. Relationships: is a type of response to chemical [GO:0042221] Sources: GOC:mah Subtypes: cellular response to anisomycin [GO:0072740]